tobramycin biosynthetic process [GO:1901121] (biological process) Also known as: tobramycin anabolism, tobramycin biosynthesis, tobramycin formation, tobramycin synthesis Definition: The chemical reactions and pathways resulting in the formation of tobramycin. Sources: GOC:TermGenie, GOC:yaf, UniPathway:UPA00971 Relationships: is a type of glycoside biosynthetic process [GO:0016138]; is a type of polyol biosynthetic process [GO:0046173]